{
  "term_id": "GO:0016094",
  "gene_name": "Dehydrodolichyl diphosphate synthase complex subunit DHDDS",
  "term_label": "polyprenol biosynthetic process",
  "gene": "UniProtKB:Q86SQ9",
  "gene_symbol": "DHDDS"
}